CDP-diacylglycerol metabolic process [GO:0046341] (biological process) Subtypes: CDP-diacylglycerol biosynthetic process [GO:0016024], CDP-diacylglycerol catabolic process [GO:0046342] References: PMID:24533860 Relationships: is a type of glycerophospholipid metabolic process [GO:0006650] Also known as: CDP-diacylglycerol metabolism Definition: The chemical reactions and pathways involving CDP-diacylglycerol, CDP-1,2-diacylglycerol, a substance composed of diacylglycerol in glycosidic linkage with cytidine diphosphate. It is a common intermediate in phospholipid biosynthesis.